voltage-gated sodium channel activity [GO:0005248] (molecular function) Definition: Enables the transmembrane transfer of a sodium ion by a voltage-gated channel. A voltage-gated channel is a channel whose open state is dependent on the voltage across the membrane in which it is embedded. Sources: GOC:mtg_transport, ISBN:0815340729 Also known as: voltage gated sodium channel activity, voltage-dependent sodium channel activity, voltage-gated sodium ion channel activity, voltage-sensitive sodium channel Relationships: is a type of sodium channel activity [GO:0005272] Subtypes: voltage-gated sodium channel activity involved in cardiac muscle cell action potential [GO:0086006], mechanosensitive voltage-gated sodium channel activity [GO:0101013] Regulation: regulated by regulation of voltage-gated sodium channel activity [GO:1905150]; positively regulated by GO:1905152